Wnt signalosome [GO:1990909] (cellular component) Relationships: is_a protein-containing complex [GO:0032991]; has part Wnt-Frizzled-LRP5/6 complex [GO:1990851] Note: Within the Wnt signalosome, beta-catenin phosphorylation is inhibited through internalization of the signalosome complex, resulting in the sequestration of GSK3-beta into multi-vesicular bodies. No longer phosphorylated and targeted for degradation, beta-catenin is free to enter the nucleus and modulate downstream transcription. Also known as: LRP5/6 signalosome, Wnt signalosome complex, Wnt-LRP5/6 signalosome, LRP6 signalosome Definition: A multiprotein protein complex containing membrane-localized Wnt receptors and cytosolic protein complexes, which is capable of transmitting the Wnt signal. Contains at least a Wnt protein, LRP5 or LRP6, a member of the Frizzled (Fz) family, Axin and and a Dishevelled (DVL) protein. References: PMID:22899650, PMID:25336320 Sources: GOC:PARL, GOC:bf